{
  "gene_symbol": "KIR3DP1",
  "gene_name": "Killer cell immunoglobulin-like receptor, three Ig domains pseudogene 1",
  "gene": "UniProtKB:A0A0G2JN01",
  "term_id": "GO:0140375",
  "term_label": "immune receptor activity"
}